{
  "term_label": "endocytosis",
  "gene_name": "Casein kinase I isoform gamma-3",
  "gene": "UniProtKB:Q9Y6M4",
  "term_id": "GO:0006897",
  "gene_symbol": "CSNK1G3"
}